{
  "gene_name": "Ephrin type-A receptor 5",
  "term_id": "GO:0005005",
  "gene": "UniProtKB:P54756",
  "term_label": "transmembrane-ephrin receptor activity",
  "gene_symbol": "EPHA5"
}